{
  "term_label": "nucleus",
  "gene_name": "ETS homologous factor",
  "gene_symbol": "EHF",
  "term_id": "GO:0005634",
  "gene": "UniProtKB:Q9NZC4"
}